{
  "term_label": "Unknown cellular component",
  "gene_name": "Coiled-coil domain-containing protein 22",
  "gene_symbol": "CCDC22",
  "gene": "UniProtKB:O60826",
  "term_id": "UNKNOWN:0003"
}